{
  "gene_name": "WD repeat-containing protein 19",
  "term_label": "Unknown molecular function",
  "term_id": "UNKNOWN:0001",
  "gene_symbol": "WDR19",
  "gene": "UniProtKB:Q8NEZ3"
}